neural plate formation [GO:0021990] (BP) Definition: The formation of the flat, thickened layer of ectodermal cells known as the neural plate. The underlying dorsal mesoderm signals the ectodermal cells above it to elongate into columnar neural plate cells. The neural plate subsequently develops into the neural tube, which gives rise to the central nervous system. References: PMID:15806586 Sources: GOC:cls, GOC:dgh, GOC:dph, GOC:jid, GO_REF:0000021 Relationships: is a type of anatomical structure formation involved in morphogenesis [GO:0048646]; is part of neural plate morphogenesis [GO:0001839]